detection of phosphate ion [GO:0010247] (biological process) Also known as: phosphate ion detection, phosphate ion perception, phosphate ion sensing Definition: The series of events in which a phosphate ion stimulus is received by a cell and converted into a molecular signal. Sources: GOC:sm Relationships: is_a GO:0009593